{
  "gene": "UniProtKB:A6NGQ2",
  "gene_name": "Oocyte-expressed protein homolog",
  "term_id": "GO:0009880",
  "gene_symbol": "OOEP",
  "term_label": "embryonic pattern specification"
}